{
  "term_id": "GO:0004984",
  "gene": "UniProtKB:Q8NGN0",
  "term_label": "olfactory receptor activity",
  "gene_symbol": "OR4D5",
  "gene_name": "Olfactory receptor 4D5"
}